{
  "gene": "UniProtKB:Q92670",
  "term_label": "Unknown cellular component",
  "term_id": "UNKNOWN:0003",
  "gene_symbol": "ZNF75CP",
  "gene_name": "Putative zinc finger protein 75C"
}